{
  "gene": "UniProtKB:Q9UBX3",
  "gene_symbol": "SLC25A10",
  "term_id": "GO:0015131",
  "term_label": "oxaloacetate transmembrane transporter activity",
  "gene_name": "Mitochondrial dicarboxylate carrier"
}